{
  "term_label": "DUBm complex",
  "gene_symbol": "ENY2",
  "gene": "UniProtKB:Q9NPA8",
  "gene_name": "Transcription and mRNA export factor ENY2",
  "term_id": "GO:0071819"
}